{
  "term_label": "potassium channel regulator activity",
  "term_id": "GO:0015459",
  "gene_name": "Potassium voltage-gated channel subfamily G member 2",
  "gene": "UniProtKB:Q9UJ96",
  "gene_symbol": "KCNG2"
}